{
  "gene_symbol": "GPR6",
  "term_id": "GO:0007189",
  "term_label": "adenylate cyclase-activating G protein-coupled receptor signaling pathway",
  "gene_name": "G-protein coupled receptor 6",
  "gene": "UniProtKB:P46095"
}